biofilm matrix [GO:0062039] (CC) Subtypes: fungal biofilm matrix [GO:0062040], GO:0097311 Relationships: is a type of specialized extracellular matrix [GO:0140047] Definition: A type of extracellular matrix that surrounds the cells within a microbial biofilm. The matrix is composed of extracellular polymeric substances including exopolysaccharides, proteins, nucleic acids, lipids, and other biomolecules. References: PMID:22571672, PMID:27129222, PMID:28516088, PMID:32663461